{
  "gene": "UniProtKB:Q9UIK5",
  "term_label": "extracellular region",
  "gene_name": "Tomoregulin-2",
  "gene_symbol": "TMEFF2",
  "term_id": "GO:0005576"
}